{
  "gene_symbol": "CEMIP",
  "gene_name": "Cell migration-inducing and hyaluronan-binding protein",
  "term_id": "UNKNOWN:0002",
  "gene": "UniProtKB:Q8WUJ3",
  "term_label": "Unknown biological process"
}